amphisome membrane [GO:1904930] (cellular component) References: PMID:17984323 Sources: GOC:TermGenie, GOC:bhm, GO_REF:0000064 Relationships: is a type of autophagosome membrane [GO:0000421]; BFO_0000050 amphisome [GO:0044753] Definition: Any membrane that is part of an amphisome.